fructose 2,6-bisphosphate metabolic process [GO:0006003] (biological process) Definition: The chemical reactions and pathways involving fructose 2,6-bisphosphate. The D enantiomer is an important regulator of the glycolytic and gluconeogenic pathways. It inhibits fructose 1,6-bisphosphatase and activates phosphofructokinase. Sources: ISBN:0198506732 Also known as: fructose 2,6-bisphosphate metabolism Relationships: is a type of phosphate-containing compound metabolic process [GO:0006796]; is a type of organophosphate metabolic process [GO:0019637]; is a type of GO:1901135